putrescine--2-oxoglutarate transaminase activity [GO:0033094] (molecular function) Definition: Catalysis of the reaction: putrescine + 2-oxoglutarate = L-glutamate + 1-pyrroline + H2O. The enzymatic part of the reaction produces 4-aminobutanal that spontaneously cyclizes to form 1-pyrroline. Relationships: is a type of GO:0008483 Sources: EC:2.6.1.82, GOC:mlg, RHEA:12268 Also known as: putrescine aminotransferase activity, putrescine transaminase activity, PAT activity, YgjG, butane-1,4-diamine:2-oxoglutarate aminotransferase activity, putrescine-alpha-ketoglutarate transaminase activity, putrescine:2-oxoglutarate aminotransferase activity, putrescine:alpha-ketoglutarate aminotransferase activity